{
  "gene_symbol": "ADCY7",
  "gene_name": "Adenylate cyclase type 7",
  "term_id": "GO:0006171",
  "term_label": "cAMP biosynthetic process",
  "gene": "UniProtKB:P51828"
}